{
  "gene": "UniProtKB:Q7L0Y3",
  "term_id": "GO:0005739",
  "gene_name": "tRNA methyltransferase 10 homolog C",
  "term_label": "mitochondrion",
  "gene_symbol": "TRMT10C"
}